{
  "term_id": "GO:0005737",
  "gene_name": "TRAF2 and NCK-interacting protein kinase",
  "term_label": "cytoplasm",
  "gene_symbol": "TNIK",
  "gene": "UniProtKB:Q9UKE5"
}